{
  "term_id": "UNKNOWN:0001",
  "term_label": "Unknown molecular function",
  "gene_symbol": "TMEM62",
  "gene": "UniProtKB:Q0P6H9",
  "gene_name": "Transmembrane protein 62"
}